{
  "gene_name": "Eukaryotic translation initiation factor 5",
  "term_id": "GO:0005829",
  "gene": "UniProtKB:P55010",
  "gene_symbol": "EIF5",
  "term_label": "cytosol"
}